{
  "gene": "UniProtKB:Q9Y228",
  "term_id": "GO:0002753",
  "term_label": "cytoplasmic pattern recognition receptor signaling pathway",
  "gene_symbol": "TRAF3IP3",
  "gene_name": "TRAF3-interacting JNK-activating modulator"
}